{
  "term_label": "nucleus",
  "gene_name": "Cullin-4A",
  "term_id": "GO:0005634",
  "gene_symbol": "CUL4A",
  "gene": "UniProtKB:Q13619"
}